positive regulation of autophagy [GO:0010508] (biological process) Subtypes: positive regulation of macroautophagy [GO:0016239], positive regulation of autophagy in response to ER overload [GO:0034263], GO:1903599, positive regulation of chaperone-mediated autophagy [GO:1904716] Relationships: is_a positive regulation of catabolic process [GO:0009896]; is a type of regulation of autophagy [GO:0010506]; positively regulates autophagy [GO:0006914] Sources: GOC:dph, GOC:tb Definition: Any process that activates, maintains or increases the rate of autophagy. Autophagy is the process in which cells digest parts of their own cytoplasm.